{
  "gene_name": "Myotrophin",
  "term_id": "GO:0005737",
  "term_label": "cytoplasm",
  "gene": "UniProtKB:P58546",
  "gene_symbol": "MTPN"
}